{
  "term_id": "GO:0006281",
  "gene_name": "SOSS complex subunit C",
  "term_label": "DNA repair",
  "gene_symbol": "INIP",
  "gene": "UniProtKB:Q9NRY2"
}